{
  "gene_symbol": "YWHAG",
  "gene_name": "14-3-3 protein gamma",
  "gene": "UniProtKB:P61981",
  "term_label": "signal transduction",
  "term_id": "GO:0007165"
}